{
  "term_id": "GO:1902775",
  "term_label": "mitochondrial large ribosomal subunit assembly",
  "gene_name": "Probable ATP-dependent RNA helicase DDX28",
  "gene_symbol": "DDX28",
  "gene": "UniProtKB:Q9NUL7"
}